{
  "gene": "UniProtKB:Q96AT9",
  "gene_symbol": "RPE",
  "term_label": "metal ion binding",
  "gene_name": "Ribulose-phosphate 3-epimerase",
  "term_id": "GO:0046872"
}